platelet activating factor receptor activity [GO:0004992] (molecular function) Sources: GOC:mah Relationships: is a type of G protein-coupled receptor activity [GO:0004930] Definition: Combining with platelet activating factor to initiate a change in cell activity. Also known as: PAF receptor activity